{
  "gene": "UniProtKB:Q96P09",
  "gene_name": "Baculoviral IAP repeat-containing protein 8",
  "term_label": "positive regulation of canonical Wnt signaling pathway",
  "gene_symbol": "BIRC8",
  "term_id": "GO:0090263"
}